{
  "gene_symbol": "CHRDL2",
  "term_id": "UNKNOWN:0003",
  "gene": "UniProtKB:Q6WN34",
  "gene_name": "Chordin-like protein 2",
  "term_label": "Unknown cellular component"
}